{
  "gene": "UniProtKB:Q6DKI7",
  "term_id": "GO:0050860",
  "term_label": "negative regulation of T cell receptor signaling pathway",
  "gene_symbol": "PVRIG",
  "gene_name": "Transmembrane protein PVRIG"
}